{
  "gene": "UniProtKB:Q8NH89",
  "term_label": "G protein-coupled receptor signaling pathway",
  "term_id": "GO:0007186",
  "gene_symbol": "OR5AK3P",
  "gene_name": "Putative olfactory receptor 5AK3"
}